{
  "gene": "UniProtKB:A0A0J9YW14",
  "gene_symbol": "IGHJ3",
  "gene_name": "Immunoglobulin heavy joining 3 (Fragment)",
  "term_label": "Unknown molecular function",
  "term_id": "UNKNOWN:0001"
}